{
  "term_id": "UNKNOWN:0002",
  "term_label": "Unknown biological process",
  "gene": "UniProtKB:Q9NWV4",
  "gene_name": "CXXC motif containing zinc binding protein",
  "gene_symbol": "CZIB"
}